phosphopantetheine-dependent carrier activity [GO:0140414] (molecular function) Definition: Binding a substrate via a thioester at the terminal thiol of a covalentely linked phosphopantetheine prosthetic group and mediating protein-protein interactions with cognate enzymes for processing or offloading of the thiol-bound substrate. Also known as: carrier protein activity Subtypes: acyl carrier activity [GO:0000036], D-alanyl carrier activity [GO:0036370] Relationships: is a type of molecular carrier activity [GO:0140104] References: PMID:17502372